galactoside O-acetyltransferase activity [GO:0008870] (molecular function) Sources: EC:2.3.1.18 Relationships: is a type of O-acetyltransferase activity [GO:0016413] Also known as: acetyl-CoA:beta-D-galactoside 6-acetyltransferase activity, galactoside acetyltransferase activity, thiogalactoside acetyltransferase activity, thiogalactoside transacetylase activity Definition: Catalysis of the reaction: acetyl-CoA + a beta-D-galactoside = CoA + a 6-acetyl-beta-D-galactoside.